{
  "term_id": "GO:0006511",
  "gene_symbol": "RNF133",
  "term_label": "ubiquitin-dependent protein catabolic process",
  "gene_name": "E3 ubiquitin-protein ligase RNF133",
  "gene": "UniProtKB:Q8WVZ7"
}